{
  "term_label": "proline-tRNA ligase activity",
  "term_id": "GO:0004827",
  "gene_symbol": "PARS2",
  "gene_name": "Probable proline--tRNA ligase, mitochondrial",
  "gene": "UniProtKB:Q7L3T8"
}